{
  "gene_symbol": "PIWIL3",
  "term_id": "GO:0007283",
  "gene_name": "Piwi-like protein 3",
  "gene": "UniProtKB:Q7Z3Z3",
  "term_label": "spermatogenesis"
}